{
  "gene": "UniProtKB:Q8TBF8",
  "term_label": "Unknown molecular function",
  "gene_symbol": "FAM81A",
  "gene_name": "Protein FAM81A",
  "term_id": "UNKNOWN:0001"
}